{
  "gene_name": "Ephrin type-B receptor 1",
  "term_id": "GO:0030425",
  "gene_symbol": "EPHB1",
  "term_label": "dendrite",
  "gene": "UniProtKB:P54762"
}